{
  "term_id": "GO:0043531",
  "term_label": "ADP binding",
  "gene_symbol": "PGK2",
  "gene": "UniProtKB:P07205",
  "gene_name": "Phosphoglycerate kinase 2"
}